{
  "gene_name": "Zinc finger protein 792",
  "term_id": "GO:0000978",
  "gene": "UniProtKB:Q3KQV3",
  "term_label": "RNA polymerase II cis-regulatory region sequence-specific DNA binding",
  "gene_symbol": "ZNF792"
}